{
  "term_label": "plasma membrane",
  "term_id": "GO:0005886",
  "gene_name": "Radixin",
  "gene_symbol": "RDX",
  "gene": "UniProtKB:P35241"
}